{
  "gene_name": "PDZ domain-containing protein 4",
  "term_label": "Unknown cellular component",
  "gene_symbol": "PDZD4",
  "gene": "UniProtKB:Q76G19",
  "term_id": "UNKNOWN:0003"
}